{
  "gene_name": "Ataxin-1-like",
  "gene": "UniProtKB:P0C7T5",
  "gene_symbol": "ATXN1L",
  "term_label": "RNA binding",
  "term_id": "GO:0003723"
}